{
  "term_id": "GO:0004930",
  "term_label": "G protein-coupled receptor activity",
  "gene": "UniProtKB:Q49SQ1",
  "gene_symbol": "GPR33",
  "gene_name": "Probable G-protein coupled receptor 33"
}